{
  "term_id": "GO:0001574",
  "gene": "UniProtKB:Q00973",
  "term_label": "ganglioside biosynthetic process",
  "gene_name": "Beta-1,4 N-acetylgalactosaminyltransferase 1",
  "gene_symbol": "B4GALNT1"
}